integument development [GO:0080060] (biological process) References: PMID:19054366 Sources: PO:0020021 Definition: The process whose specific outcome is the progression of the integument over time, from its formation to the mature structure. Integument is one of the layers of tissue that usually covers the ovule, enveloping the nucellus and forming the micropyle at the apex. Relationships: is a type of developmental process involved in reproduction [GO:0003006]; is a type of tissue development [GO:0009888]; BFO_0000050 plant ovule development [GO:0048481]